{
  "term_id": "GO:0033617",
  "gene": "UniProtKB:Q5RI15",
  "gene_name": "Cytochrome c oxidase assembly protein COX20, mitochondrial",
  "term_label": "mitochondrial respiratory chain complex IV assembly",
  "gene_symbol": "COX20"
}